{
  "term_id": "GO:0032982",
  "gene_symbol": "MYO18A",
  "gene_name": "Unconventional myosin-XVIIIa",
  "term_label": "myosin filament",
  "gene": "UniProtKB:Q92614"
}